{
  "gene": "UniProtKB:P52741",
  "term_id": "GO:0002682",
  "term_label": "regulation of immune system process",
  "gene_symbol": "ZNF134",
  "gene_name": "Zinc finger protein 134"
}